{
  "term_label": "Unknown molecular function",
  "term_id": "UNKNOWN:0001",
  "gene_name": "Neurogranin",
  "gene": "UniProtKB:Q92686",
  "gene_symbol": "NRGN"
}